{
  "term_id": "GO:0005886",
  "term_label": "plasma membrane",
  "gene": "UniProtKB:O60500",
  "gene_name": "Nephrin",
  "gene_symbol": "NPHS1"
}